dibasic protein processing [GO:0090472] (BP) Sources: GOC:al Relationships: is_a protein processing [GO:0016485] Subtypes: lys-arg specific dibasic protein processing [GO:0090473], arg-arg specific dibasic protein processing [GO:0090474], lys-lys specific dibasic protein processing [GO:0090475] Definition: Any protein processing achieved by the cleavage of a peptide bond after two basic amino acids within a protein.